{
  "gene": "UniProtKB:Q2M1P5",
  "term_id": "GO:0008017",
  "gene_name": "Kinesin-like protein KIF7",
  "gene_symbol": "KIF7",
  "term_label": "microtubule binding"
}